{
  "gene": "UniProtKB:Q96E29",
  "gene_name": "Transcription termination factor 3, mitochondrial",
  "term_id": "GO:0005739",
  "gene_symbol": "MTERF3",
  "term_label": "mitochondrion"
}